{
  "term_label": "6-phosphofructokinase activity",
  "gene_symbol": "PFKM",
  "term_id": "GO:0003872",
  "gene": "UniProtKB:P08237",
  "gene_name": "ATP-dependent 6-phosphofructokinase, muscle type"
}